lysophospholipid acyltransferase activity [GO:0071617] (molecular function) Definition: Catalysis of the transfer of acyl groups from an acyl-CoA to a lysophospholipid. Sources: GOC:cjk Relationships: is a type of acyltransferase activity, transferring groups other than amino-acyl groups [GO:0016747] Subtypes: GO:0042171, lysophosphatidylethanolamine acyltransferase activity [GO:0071618]